{
  "term_id": "GO:0070888",
  "gene_symbol": "NEUROD2",
  "term_label": "E-box binding",
  "gene": "UniProtKB:Q15784",
  "gene_name": "Neurogenic differentiation factor 2"
}